{
  "term_id": "GO:0030178",
  "gene_name": "Protein chibby homolog 1",
  "gene": "UniProtKB:Q9Y3M2",
  "gene_symbol": "CBY1",
  "term_label": "negative regulation of Wnt signaling pathway"
}